{
  "term_id": "GO:0009897",
  "gene_symbol": "FCRL1",
  "term_label": "external side of plasma membrane",
  "gene_name": "Fc receptor-like protein 1",
  "gene": "UniProtKB:Q96LA6"
}